{
  "gene": "UniProtKB:O75419",
  "gene_symbol": "CDC45",
  "gene_name": "Cell division control protein 45 homolog",
  "term_id": "GO:0003682",
  "term_label": "chromatin binding"
}